{
  "gene_symbol": "ADGRB2",
  "term_id": "GO:0007186",
  "term_label": "G protein-coupled receptor signaling pathway",
  "gene": "UniProtKB:O60241",
  "gene_name": "Adhesion G protein-coupled receptor B2"
}